{
  "gene": "UniProtKB:Q5T1J6",
  "gene_name": "Protein FAM182A",
  "gene_symbol": "FAM182A",
  "term_id": "UNKNOWN:0002",
  "term_label": "Unknown biological process"
}